{
  "term_label": "DNA-binding transcription factor activity, RNA polymerase II-specific",
  "gene_symbol": "PLAG1",
  "term_id": "GO:0000981",
  "gene": "UniProtKB:Q6DJT9",
  "gene_name": "Zinc finger protein PLAG1"
}